beta-2-microglobulin binding [GO:0030881] (molecular function) Definition: Binding to beta-2-microglobulin. Sources: GOC:mah Relationships: is a type of GO:0005515